{
  "gene_symbol": "OAZ1",
  "term_label": "ornithine decarboxylase inhibitor activity",
  "term_id": "GO:0008073",
  "gene": "UniProtKB:P54368",
  "gene_name": "Ornithine decarboxylase antizyme 1"
}